{
  "term_label": "microtubule end",
  "term_id": "GO:1990752",
  "gene_name": "Neuron navigator 3",
  "gene": "UniProtKB:Q8IVL0",
  "gene_symbol": "NAV3"
}